{
  "gene": "UniProtKB:Q9Y312",
  "gene_symbol": "AAR2",
  "gene_name": "Protein AAR2 homolog",
  "term_label": "Unknown cellular component",
  "term_id": "UNKNOWN:0003"
}